uterine wall breakdown [GO:0042704] (biological process) Relationships: is a type of ovulation cycle process [GO:0022602]; happens during menstruation [GO:0042703] Sources: GOC:dph Definition: The sloughing of the endometrium and blood vessels during menstruation that results from a drop in progesterone levels.